{
  "term_id": "UNKNOWN:0001",
  "term_label": "Unknown molecular function",
  "gene": "UniProtKB:Q5TA79",
  "gene_name": "Late cornified envelope protein 2A",
  "gene_symbol": "LCE2A"
}